{
  "gene": "UniProtKB:Q02325",
  "gene_name": "Plasminogen-like protein B",
  "term_label": "Unknown biological process",
  "term_id": "UNKNOWN:0002",
  "gene_symbol": "PLGLB2"
}